{
  "term_label": "Unknown biological process",
  "gene_name": "PHD finger protein 14",
  "gene": "UniProtKB:O94880",
  "term_id": "UNKNOWN:0002",
  "gene_symbol": "PHF14"
}